{
  "gene": "UniProtKB:P50749",
  "term_id": "UNKNOWN:0001",
  "term_label": "Unknown molecular function",
  "gene_symbol": "RASSF2",
  "gene_name": "Ras association domain-containing protein 2"
}